positive regulation of maintenance of sister chromatid cohesion [GO:0034093] (biological process) Relationships: is a type of GO:0034091; is a type of positive regulation of sister chromatid cohesion [GO:0045876]; positively regulates GO:0034086 Definition: Any process that increases the extent to which the association between sister chromatids of a replicated chromosome is maintained. Sources: GOC:mah, GOC:vw Subtypes: positive regulation of maintenance of meiotic sister chromatid cohesion [GO:0034096], positive regulation of maintenance of mitotic sister chromatid cohesion [GO:0034184]